{
  "term_label": "olfactory receptor activity",
  "gene_name": "Olfactory receptor 8A1",
  "gene": "UniProtKB:Q8NGG7",
  "term_id": "GO:0004984",
  "gene_symbol": "OR8A1"
}